{
  "gene_symbol": "TASOR2",
  "term_label": "nucleoplasm",
  "gene_name": "Protein TASOR 2",
  "term_id": "GO:0005654",
  "gene": "UniProtKB:Q5VWN6"
}